intracellular protein transmembrane transport [GO:0065002] (biological process) Also known as: intracellular membrane translocation of a protein, intracellular protein membrane transport, intracellular protein transport across a membrane Definition: The directed movement of proteins in a cell, from one side of a membrane to another by means of some agent such as a transporter or pore. Note: Note that this term is not intended for use in annotating lateral movement within membranes. Relationships: is a type of GO:0006886; is a type of protein transmembrane transport [GO:0071806] Sources: GOC:isa_complete Subtypes: SRP-dependent cotranslational protein targeting to membrane, translocation [GO:0006616], protein import into peroxisome matrix, translocation [GO:0016561], post-translational protein targeting to membrane, translocation [GO:0031204], protein transmembrane import into intracellular organelle [GO:0044743]